{
  "term_label": "DNA-binding transcription factor activity, RNA polymerase II-specific",
  "gene": "UniProtKB:Q9H9S0",
  "term_id": "GO:0000981",
  "gene_name": "Homeobox protein NANOG",
  "gene_symbol": "NANOG"
}